{
  "gene": "UniProtKB:Q9BWW4",
  "gene_name": "Single-stranded DNA-binding protein 3",
  "term_label": "positive regulation of transcription by RNA polymerase II",
  "gene_symbol": "SSBP3",
  "term_id": "GO:0045944"
}